{
  "gene_name": "Voltage-dependent calcium channel subunit alpha-2_delta-3",
  "gene_symbol": "CACNA2D3",
  "gene": "UniProtKB:Q8IZS8",
  "term_id": "GO:0005245",
  "term_label": "voltage-gated calcium channel activity"
}